{
  "gene": "UniProtKB:Q6ZN18",
  "term_id": "GO:0035098",
  "gene_name": "Zinc finger protein AEBP2",
  "gene_symbol": "AEBP2",
  "term_label": "ESC/E(Z) complex"
}